{
  "gene_name": "Activator of basal transcription 1",
  "term_label": "endonucleolytic cleavage in 5'-ETS of tricistronic rRNA transcript (SSU-rRNA, 5.8S rRNA, LSU-rRNA)",
  "gene_symbol": "ABT1",
  "term_id": "GO:0000480",
  "gene": "UniProtKB:Q9ULW3"
}